{
  "gene_symbol": "POP1",
  "gene_name": "Ribonucleases P_MRP protein subunit POP1",
  "gene": "UniProtKB:Q99575",
  "term_id": "GO:0005655",
  "term_label": "nucleolar ribonuclease P complex"
}